negative regulation of purine nucleotide biosynthetic process [GO:1900372] (BP) Relationships: is a type of negative regulation of nucleotide biosynthetic process [GO:0030809]; is_a regulation of purine nucleotide biosynthetic process [GO:1900371]; is_a negative regulation of purine nucleotide metabolic process [GO:1900543]; negatively regulates GO:0006164 Sources: GOC:TermGenie, GOC:go_curators Also known as: down regulation of purine nucleotide anabolism, down regulation of purine nucleotide biosynthesis, down regulation of purine nucleotide biosynthetic process, down regulation of purine nucleotide formation, down regulation of purine nucleotide synthesis, down-regulation of purine nucleotide anabolism, down-regulation of purine nucleotide biosynthesis, down-regulation of purine nucleotide biosynthetic process, down-regulation of purine nucleotide formation, down-regulation of purine nucleotide synthesis, downregulation of purine nucleotide anabolism, downregulation of purine nucleotide biosynthesis, downregulation of purine nucleotide biosynthetic process, downregulation of purine nucleotide formation, downregulation of purine nucleotide synthesis, inhibition of purine nucleotide anabolism, inhibition of purine nucleotide biosynthesis, inhibition of purine nucleotide formation, inhibition of purine nucleotide synthesis, negative regulation of purine nucleotide anabolism, negative regulation of purine nucleotide biosynthesis, negative regulation of purine nucleotide formation, negative regulation of purine nucleotide synthesis, inhibition of purine nucleotide biosynthetic process Definition: Any process that stops, prevents or reduces the frequency, rate or extent of purine nucleotide biosynthetic processes. Subtypes: negative regulation of guanylate cyclase activity [GO:0031283], negative regulation of 'de novo' NAD biosynthetic process from L-tryptophan [GO:1905013], GO:2001170